RNAi-mediated antiviral immunity against RNA virus [GO:0051214] (biological process) Definition: An RNAi-mediated post-transcriptional gene silencing pathway induced by RNA viruses leading to a sequence-specific degradation of target mRNAs or inhibition of translation. In plants, DCL4 is the primary Dicer to detect RNA viruses. Relationships: is a type of RNAi-mediated antiviral immune response [GO:0009616] Also known as: RNA VIGS, RNA virus induced gene silencing, RNA virus-induced PTGS, RNA virus-induced gene silencing References: PMID:15165191, PMID:17693253